{
  "gene_name": "NKAP-like protein",
  "gene_symbol": "NKAPL",
  "gene": "UniProtKB:Q5M9Q1",
  "term_id": "GO:0010468",
  "term_label": "regulation of gene expression"
}